{
  "term_label": "C-C chemokine binding",
  "gene_name": "C-C chemokine receptor type 4",
  "term_id": "GO:0019957",
  "gene": "UniProtKB:P51679",
  "gene_symbol": "CCR4"
}